cyanidin 3-O-glucoside 5-O-glucosyltransferase (acyl-glucose) activity [GO:0102506] (molecular function) Relationships: is a type of GO:0016758 Sources: RHEA:35427 Definition: Catalysis of the reaction: cyanidin 3-O-beta-D-glucoside betaine + 1-O-feruloyl-beta-D-glucose = cyanin betaine + ferulate + H+.